{
  "gene": "UniProtKB:Q8IYX3",
  "gene_symbol": "CCDC116",
  "term_label": "centrosome",
  "gene_name": "Coiled-coil domain-containing protein 116",
  "term_id": "GO:0005813"
}